{
  "term_label": "cytoplasm",
  "term_id": "GO:0005737",
  "gene": "UniProtKB:Q8NDN9",
  "gene_name": "RCC1 and BTB domain-containing protein 1",
  "gene_symbol": "RCBTB1"
}